{
  "term_id": "GO:0004896",
  "term_label": "cytokine receptor activity",
  "gene_symbol": "CRLF2",
  "gene_name": "Cytokine receptor-like factor 2",
  "gene": "UniProtKB:Q9HC73"
}